{
  "gene_name": "Translocon-associated protein subunit beta",
  "gene_symbol": "SSR2",
  "term_label": "Unknown biological process",
  "gene": "UniProtKB:P43308",
  "term_id": "UNKNOWN:0002"
}